{
  "gene_name": "Serine_threonine-protein kinase pim-3",
  "term_id": "GO:0005737",
  "gene_symbol": "PIM3",
  "gene": "UniProtKB:Q86V86",
  "term_label": "cytoplasm"
}